{
  "term_label": "Unknown molecular function",
  "gene": "UniProtKB:Q9H8P0",
  "gene_symbol": "SRD5A3",
  "term_id": "UNKNOWN:0001",
  "gene_name": "Polyprenol reductase"
}